amino acid adenylylation by nonribosomal peptide synthase [GO:0043042] (biological process) Relationships: is a type of amino acid activation for nonribosomal peptide biosynthetic process [GO:0043041] Also known as: amino acid adenylation by NRPS, amino acid adenylation by nonribosomal peptide synthase References: PMID:9250661, PMID:9712910 Sources: GOC:jl Definition: Activation of an amino acid for incorporation into a peptide by a nonribosomal process, catalyzed by subunits of nonribosomal peptide synthase. The amino acid is adenylated at its carboxylate group (ATP-dependent) then transferred to the thiol group of an enzyme-bound phosphopantetheine cofactor.